{
  "gene_name": "Receptor activity-modifying protein 1",
  "gene_symbol": "RAMP1",
  "term_label": "calcium ion transport",
  "gene": "UniProtKB:O60894",
  "term_id": "GO:0006816"
}